regulation of axon guidance [GO:1902667] (biological process) Also known as: regulation of axon pathfinding, regulation of axon growth cone guidance, regulation of axon chemotaxis Subtypes: GO:0090259, negative regulation of axon guidance [GO:1902668], positive regulation of axon guidance [GO:1902669], regulation of anterior/posterior axon guidance [GO:1905486], regulation of sensory neuron axon guidance [GO:1905489], GO:1905812, regulation of dorsal/ventral axon guidance [GO:1905815], regulation of photoreceptor cell axon guidance [GO:2000289] References: PMID:23006775 Sources: GOC:TermGenie, GOC:hjd, GO_REF:0000058 Definition: Any process that modulates the frequency, rate or extent of axon guidance. Relationships: is a type of GO:0010975; is a type of GO:0050920; regulates axon guidance [GO:0007411]